{
  "term_id": "GO:0046856",
  "gene": "UniProtKB:Q92562",
  "gene_symbol": "FIG4",
  "gene_name": "Polyphosphoinositide phosphatase",
  "term_label": "phosphatidylinositol dephosphorylation"
}